{
  "term_id": "GO:0061630",
  "gene": "UniProtKB:Q9NYG5",
  "gene_symbol": "ANAPC11",
  "term_label": "ubiquitin protein ligase activity",
  "gene_name": "Anaphase-promoting complex subunit 11"
}